{
  "term_id": "GO:0042564",
  "gene_name": "Importin subunit alpha-4",
  "term_label": "NLS-dependent protein nuclear import complex",
  "gene": "UniProtKB:O00505",
  "gene_symbol": "KPNA3"
}